hydrolase activity, acting on carbon-nitrogen (but not peptide) bonds, in linear amides [GO:0016811] (molecular function) Relationships: is_a GO:0016810 Definition: Catalysis of the hydrolysis of any non-peptide carbon-nitrogen bond in a linear amide. Subtypes: peptide-N4-(N-acetyl-beta-glucosaminyl)asparagine amidase activity [GO:0000224], N-acetylglucosaminylphosphatidylinositol deacetylase activity [GO:0000225], GO:0003832, beta-ureidopropionase activity [GO:0003837], N4-(beta-N-acetylglucosaminyl)-L-asparaginase activity [GO:0003948], allophanate hydrolase activity [GO:0004039], amidase activity [GO:0004040], aminoacylase activity [GO:0004046], arylformamidase activity [GO:0004061], chitin deacetylase activity [GO:0004099], GO:0004359, pantothenase activity [GO:0004593], GO:0004848, GO:0008421, N-acetylglucosamine-6-phosphate deacetylase activity [GO:0008448], formylmethionine deformylase activity [GO:0008463], GO:0008745, acetylornithine deacetylase activity [GO:0008777], formyltetrahydrofolate deformylase activity [GO:0008864], GO:0008884, penicillin amidase activity [GO:0008953], GO:0009014, succinylglutamate desuccinylase activity [GO:0009017], urease activity [GO:0009039], GO:0017040, fatty acid amide hydrolase activity [GO:0017064], pantetheine hydrolase activity [GO:0017159], biuret amidohydrolase activity [GO:0018750], GO:0019159, aspartoacylase activity [GO:0019807], 6-aminohexanoate-dimer hydrolase activity [GO:0019875], GO:0031964, GO:0033964, aculeacin-A deacylase activity [GO:0033965], GO:0033966, glutaryl-7-aminocephalosporanic-acid acylase activity [GO:0033968], gamma-glutamyl-gamma-aminobutyrate hydrolase activity [GO:0033969], N-malonylurea hydrolase activity [GO:0033970], N-acetylglucosaminylinositol deacetylase activity [GO:0035595], protein-malonyllysine demalonylase activity [GO:0036054], chitin disaccharide deacetylase activity [GO:0036311], protein deglycase activity [GO:0036524], peptide deformylase activity [GO:0042586], tubulin deacetylase activity [GO:0042903], adenosine 5'-monophosphoramidase activity [GO:0043530], 2-amino-5-formylamino-6-(5-phosphoribosylamino)pyrimidin-4(3H)-one formate-lyase activity [GO:0043729], adenosylcobinamide hydrolase activity [GO:0043756], N-acetylcitrulline deacetylase activity [GO:0043909], GO:0045302, 2-(acetamidomethylene)succinate hydrolase activity [GO:0047411], N-(long-chain-acyl)ethanolamine deacylase activity [GO:0047412], N(alpha)-benzyloxycarbonylleucine hydrolase activity [GO:0047413], 2-(hydroxymethyl)-3-(acetamidomethylene)succinate hydrolase activity [GO:0047414], D-benzoylarginine-4-nitroanilide amidase activity [GO:0047415], GO:0047416, N-carbamoyl-D-amino acid hydrolase activity [GO:0047417], GO:0047418, N-acetylgalactosamine-6-phosphate deacetylase activity [GO:0047419], GO:0047420, N-acyl-D-glutamate deacylase activity [GO:0047421], N-acyl-D-aspartate deacylase activity [GO:0047422], 4-acetamidobutyrate deacetylase activity [GO:0047573], 4-acetamidobutyryl-CoA deacetylase activity [GO:0047574], GO:0047582, 5-aminopentanamidase activity [GO:0047588], acetylputrescine deacetylase activity [GO:0047609], acetylspermidine deacetylase activity [GO:0047611], acylagmatine amidase activity [GO:0047618], alkylamidase activity [GO:0047648], GO:0047680, GO:0047708, GO:0047742, GO:0047773, citrullinase activity [GO:0047781], formylaspartate deformylase activity [GO:0047902], GO:0047980, D-glutaminase activity [GO:0050001], N,N-dimethylformamidase activity [GO:0050116], GO:0050117, N-acetyldiaminopimelate deacetylase activity [GO:0050118], N-acetylglucosamine deacetylase activity [GO:0050119], N-benzyloxycarbonylglycine hydrolase activity [GO:0050125], N-carbamoylputrescine amidase activity [GO:0050126], N-carbamoylsarcosine amidase activity [GO:0050127], N-feruloylglycine deacylase activity [GO:0050128], N-formylglutamate deformylase activity [GO:0050129], N-methyl-2-oxoglutaramate hydrolase activity [GO:0050130], omega-amidase activity [GO:0050152], pentanamidase activity [GO:0050168], GO:0050170, theanine hydrolase activity [GO:0050330], GO:0050365, ureidosuccinase activity [GO:0050386], urethanase activity [GO:0050387], glutamin-(asparagin-)ase activity [GO:0050417], acyl-lysine deacylase activity [GO:0050477], (S)-N-acetyl-1-phenylethylamine hydrolase activity [GO:0050536], mandelamide amidase activity [GO:0050537], N-carbamoyl-L-amino-acid hydrolase activity [GO:0050538], protein-glutamine glutaminase activity [GO:0050568], GO:0052773, GO:0061690, protein-N-terminal glutamine amidohydrolase activity [GO:0070773], para-aminobenzoyl-glutamate hydrolase activity [GO:0071713], GO:0102572, UDP-3-O-acyl-N-acetylglucosamine deacetylase activity [GO:0103117], 2-oxoglutaramate amidase activity [GO:0106008], GO:0106251, deaminated glutathione amidase activity [GO:0110050], GO:0141221, protein decrotonylase activity [GO:0160008], protein de-2-hydroxyisobutyrylase activity [GO:0160010], protein asparagine deamidase activity [GO:0160260], amino acid conjugated cholate hydrolase activity [GO:7770003] Sources: EC:3.5.1.-